{
  "gene_name": "Allograft inflammatory factor 1-like",
  "term_label": "actin filament binding",
  "term_id": "GO:0051015",
  "gene": "UniProtKB:Q9BQI0",
  "gene_symbol": "AIF1L"
}